repressor ecdysone receptor complex [GO:0008231] (cellular component) Relationships: is a type of ecdysone receptor holocomplex [GO:0008230] References: PMID:10488333 Definition: A protein complex consisting of a heterodimer of Ecdysone receptor (EcR) and ultraspiracle (usp) plus an associated corepressor such as SMRTER, which represses transcription of target genes. Also known as: repressor ecdysone receptor holocomplex